nucleosome disassembly [GO:0006337] (biological process) Relationships: is a type of protein-DNA complex disassembly [GO:0032986]; is a type of GO:0034728 Definition: The controlled breakdown of nucleosomes, the beadlike structural units of eukaryotic chromatin composed of histones and DNA. Sources: GOC:mah